{
  "term_label": "chiasma assembly",
  "gene_name": "MutS protein homolog 5",
  "gene_symbol": "MSH5",
  "term_id": "GO:0051026",
  "gene": "UniProtKB:O43196"
}